{
  "gene_symbol": "SRFBP1",
  "gene": "UniProtKB:Q8NEF9",
  "term_id": "GO:0030686",
  "gene_name": "Serum response factor-binding protein 1",
  "term_label": "90S preribosome"
}